skeletal muscle adaptation [GO:0043501] (biological process) Definition: Any process in which skeletal muscles change their phenotypic profiles in response to altered functional demands and a variety of signals. Subtypes: GO:0014732, skeletal muscle hypertrophy [GO:0014734] Also known as: skeletal muscle plasticity Relationships: is a type of striated muscle adaptation [GO:0014888] Regulation: regulated by regulation of skeletal muscle adaptation [GO:0014733] References: PMID:11181628, PMID:11449884, PMID:12605307 Sources: GOC:mtg_muscle